{
  "gene_name": "N-terminal EF-hand calcium-binding protein 1",
  "gene_symbol": "NECAB1",
  "gene": "UniProtKB:Q8N987",
  "term_label": "Unknown molecular function",
  "term_id": "UNKNOWN:0001"
}